{
  "gene_symbol": "TMOD4",
  "term_label": "cytoskeleton",
  "gene_name": "Tropomodulin-4",
  "term_id": "GO:0005856",
  "gene": "UniProtKB:Q9NZQ9"
}